{
  "gene": "UniProtKB:Q9BPW8",
  "gene_symbol": "NIPSNAP1",
  "term_label": "sensory perception of pain",
  "gene_name": "Protein NipSnap homolog 1",
  "term_id": "GO:0019233"
}